{
  "gene_name": "Histone H2A type 1-B_E",
  "term_id": "GO:0005634",
  "gene": "UniProtKB:P04908",
  "gene_symbol": "H2AC8",
  "term_label": "nucleus"
}